(R)-mevalonic acid catabolic process [GO:1901736] (biological process) Also known as: (R)-mevalonate breakdown, (R)-mevalonate catabolism, (R)-mevalonate degradation, (R)-mevalonic acid breakdown, (R)-mevalonic acid catabolism, (R)-mevalonic acid degradation Definition: The chemical reactions and pathways resulting in the breakdown of (R)-mevalonic acid. Sources: GOC:TermGenie, GOC:yaf, UniPathway:UPA00058 Relationships: is_a GO:0072329